{
  "term_label": "Unknown molecular function",
  "gene_name": "Protein FAM185A",
  "gene": "UniProtKB:Q8N0U4",
  "term_id": "UNKNOWN:0001",
  "gene_symbol": "FAM185A"
}